tryptophan-phenylpyruvate transaminase activity [GO:0047299] (molecular function) Relationships: is_a transaminase activity [GO:0008483] Definition: Catalysis of the reaction: keto-phenylpyruvate + L-tryptophan = 3-(indol-3-yl)pyruvate + L-phenylalanine. Also known as: tryptophan-phenylpyruvate aminotransferase activity, L-tryptophan-alpha-ketoisocaproate aminotransferase activity, L-tryptophan:phenylpyruvate aminotransferase activity, tryptophan--phenylpyruvate aminotransferase activity Sources: EC:2.6.1.28, RHEA:13741